{
  "gene_name": "Metallophosphoesterase MPPED2",
  "term_id": "UNKNOWN:0002",
  "gene_symbol": "MPPED2",
  "term_label": "Unknown biological process",
  "gene": "UniProtKB:Q15777"
}